{
  "gene_symbol": "FKBP2",
  "term_id": "GO:0003755",
  "gene": "UniProtKB:P26885",
  "gene_name": "Peptidyl-prolyl cis-trans isomerase FKBP2",
  "term_label": "peptidyl-prolyl cis-trans isomerase activity"
}